acetoacetic acid biosynthetic process [GO:0043441] (BP) Relationships: is a type of acetoacetic acid metabolic process [GO:0043438]; is a type of ketone body biosynthetic process [GO:0046951]; is a type of GO:0051790 Definition: The chemical reactions and pathways resulting in the formation of acetoacetic acid, a beta-keto acid of the keto acid group, empirical formula is C4H6O3 or CH3COCH2COOH. Also known as: acetoacetic acid anabolism, acetoacetic acid biosynthesis, acetoacetic acid formation, acetoacetic acid synthesis Sources: GOC:jl